post-embryonic root development [GO:0048528] (biological process) Subtypes: lateral root development [GO:0048527] Sources: GOC:tb Relationships: is a type of GO:0048364; is a type of post-embryonic plant organ development [GO:0090696] Regulation: regulated by regulation of post-embryonic root development [GO:2000069] Definition: The process whose specific outcome is the progression of the post-embryonic root over time, from its formation to the mature structure.